{
  "term_id": "GO:0045121",
  "gene": "UniProtKB:Q9ULV8",
  "gene_symbol": "CBLC",
  "gene_name": "E3 ubiquitin-protein ligase CBL-C",
  "term_label": "membrane raft"
}